{
  "term_id": "UNKNOWN:0001",
  "gene_name": "Tumor protein D54",
  "term_label": "Unknown molecular function",
  "gene_symbol": "TPD52L2",
  "gene": "UniProtKB:O43399"
}